{
  "gene": "UniProtKB:Q8WVF1",
  "gene_name": "Protein OSCP1",
  "term_id": "GO:0005886",
  "gene_symbol": "OSCP1",
  "term_label": "plasma membrane"
}